symbiont intracellular protein transport in host [GO:0030581] (biological process) Subtypes: GO:0019060 Relationships: is a type of GO:0015031; is a type of biological process involved in interaction with host [GO:0051701]; occurs in host cell [GO:0043657] Sources: GOC:mb Definition: The directed movement of a symbiont's proteins within a cell of the host organism. The host is defined as the larger of the organisms involved in a symbiotic interaction. Also known as: intracellular protein transport in other organism during symbiotic interaction, intracellular protein transport in other organism involved in symbiotic interaction, host cell protein transport, intracellular protein transport in host